detoxification of copper ion [GO:0010273] (biological process) Definition: Any process that reduces or removes the toxicity of copper ion. These include transport of copper away from sensitive areas and to compartments or complexes whose purpose is sequestration of copper ion. References: PMID:16367966 Sources: GOC:kmv Relationships: is a type of detoxification of inorganic compound [GO:0061687]; is part of stress response to copper ion [GO:1990169] Subtypes: cellular detoxification of copper ion [GO:1990880]